{
  "term_label": "GTPase activator activity",
  "gene_symbol": "TBC1D7",
  "term_id": "GO:0005096",
  "gene": "UniProtKB:Q9P0N9",
  "gene_name": "TBC1 domain family member 7"
}